{
  "gene_name": "Protein SFI1 homolog",
  "gene": "UniProtKB:A8K8P3",
  "term_label": "phosphatase binding",
  "term_id": "GO:0019902",
  "gene_symbol": "SFI1"
}